protein-L-histidine N-tele-methyltransferase activity [GO:0018064] (molecular function) Relationships: is a type of N-methyltransferase activity [GO:0008170]; is_a protein methyltransferase activity [GO:0008276]; is a type of S-adenosylmethionine-dependent methyltransferase activity [GO:0008757] Also known as: protein-histidine N-methyltransferase activity, peptidyl-histidine N-methyltransferase activity, protein methylase IV activity, S-adenosyl methionine:protein-histidine N-methyltransferase activity, S-adenosyl-L-methionine:protein-L-histidine N-tele-methyltransferase activity, actin-specific histidine methyltransferase activity, protein (histidine) methyltransferase activity Sources: RHEA:19369 Definition: Catalysis of the reaction: L-histidyl-[protein] + S-adenosyl-L-methionine = N(tele)-methyl-L-histidyl-[protein] + S-adenosyl-L-homocysteine.